{
  "gene_name": "FAST kinase domain-containing protein 2, mitochondrial",
  "gene": "UniProtKB:Q9NYY8",
  "gene_symbol": "FASTKD2",
  "term_label": "mitochondrial RNA processing",
  "term_id": "GO:0000963"
}